{
  "gene": "UniProtKB:P06748",
  "term_label": "ribosomal small subunit biogenesis",
  "term_id": "GO:0042274",
  "gene_name": "Nucleophosmin",
  "gene_symbol": "NPM1"
}